2,4-dichlorophenoxyacetic acid metabolic process [GO:0018901] (biological process) Subtypes: GO:0046300 Relationships: is a type of GO:0032787; is a type of benzene-containing compound metabolic process [GO:0042537]; is a type of organohalogen metabolic process [GO:0090345] Also known as: 2,4-D metabolic process, 2,4-D metabolism, 2,4-dichlorophenoxyacetic acid metabolism Definition: The chemical reactions and pathways involving 2,4-dichlorophenoxyacetic acid, a chlorinated phenoxy compound which functions as a systemic herbicide and is used to control many types of broadleaf weeds. Sources: GOC:curators